{
  "term_id": "UNKNOWN:0002",
  "term_label": "Unknown biological process",
  "gene": "UniProtKB:A6NL05",
  "gene_symbol": "FAM74A7",
  "gene_name": "Protein FAM74A7"
}